{
  "gene_symbol": "MRGPRX3",
  "gene_name": "Mas-related G-protein coupled receptor member X3",
  "term_label": "G protein-coupled receptor signaling pathway",
  "term_id": "GO:0007186",
  "gene": "UniProtKB:Q96LB0"
}